{
  "gene_name": "Excitatory amino acid transporter 5",
  "term_id": "GO:0015813",
  "gene": "UniProtKB:O00341",
  "gene_symbol": "SLC1A7",
  "term_label": "L-glutamate transmembrane transport"
}